{
  "gene_symbol": "CNTN3",
  "gene": "UniProtKB:Q9P232",
  "term_id": "UNKNOWN:0001",
  "gene_name": "Contactin-3",
  "term_label": "Unknown molecular function"
}